mitochondrial ribonuclease P complex [GO:0030678] (cellular component) Relationships: is a type of ribonuclease P complex [GO:0030677]; is a type of mitochondrial protein-containing complex [GO:0098798] Definition: A ribonuclease P complex located in the mitochondrion of a eukaryotic cell, where it catalyzes the 5' endonucleolytic cleavage of precursor tRNAs to yield mature tRNAs. The subunit composition of mitochondrial ribonuclease P complexes varies between species. The complex contains a single RNA molecule and a single protein molecule in yeast (PMID:12045094), but comprises three proteins and lacks an RNA component in humans. References: PMID:12045094, PMID:27187488 Sources: GOC:mah Also known as: mitochondrial RNase P complex